{
  "gene": "UniProtKB:P40205",
  "term_id": "UNKNOWN:0003",
  "gene_name": "N-cym protein",
  "gene_symbol": "MYCNOS",
  "term_label": "Unknown cellular component"
}